pyrimidine deoxyribonucleoside diphosphate metabolic process [GO:0009196] (biological process) Relationships: is a type of GO:0009138 Sources: GOC:go_curators, ISBN:0198506732 Also known as: pyrimidine deoxyribonucleoside diphosphate metabolism Definition: The chemical reactions and pathways involving pyrimidine deoxynucleoside diphosphate, a compound consisting of a pyrimidine base linked to a deoxyribose sugar esterified with diphosphate on the sugar. Subtypes: GO:0009197, GO:0009198, GO:0046062, dTDP metabolic process [GO:0046072], dUDP metabolic process [GO:0046077]